{
  "term_label": "Unknown molecular function",
  "term_id": "UNKNOWN:0001",
  "gene_symbol": "C1orf115",
  "gene_name": "Required for drug-induced death protein 1",
  "gene": "UniProtKB:Q9H7X2"
}